{
  "gene_name": "Nicotinate phosphoribosyltransferase",
  "gene_symbol": "NAPRT",
  "gene": "UniProtKB:Q6XQN6",
  "term_label": "cytosol",
  "term_id": "GO:0005829"
}